{
  "gene_symbol": "GRHL3",
  "gene": "UniProtKB:Q8TE85",
  "term_id": "GO:0005634",
  "term_label": "nucleus",
  "gene_name": "Grainyhead-like protein 3 homolog"
}